regulation of ubiquitin-dependent protein catabolic process [GO:2000058] (biological process) Relationships: is a type of GO:0009894; is a type of regulation of proteolysis involved in protein catabolic process [GO:1903050]; regulates GO:0006511 Definition: Any process that modulates the frequency, rate or extent of ubiquitin-dependent protein catabolic process. Sources: GOC:BHF Also known as: regulation of protein ubiquitination during ubiquitin-dependent protein breakdown, regulation of protein ubiquitination during ubiquitin-dependent protein catabolism, regulation of protein ubiquitination during ubiquitin-dependent protein degradation, regulation of protein ubiquitinylation during ubiquitin-dependent protein catabolic process, regulation of protein ubiquitinylation during ubiquitin-dependent protein catabolism, regulation of protein ubiquitylation during ubiquitin-dependent protein catabolic process, regulation of protein ubiquitylation during ubiquitin-dependent protein catabolism, regulation of protein ubiquitination involved in ubiquitin-dependent protein catabolic process, regulation of myofibrillar protein ubiquitination during ubiquitin-dependent protein breakdown, regulation of myofibrillar protein ubiquitination during ubiquitin-dependent protein catabolic process, regulation of myofibrillar protein ubiquitination during ubiquitin-dependent protein catabolism, regulation of myofibrillar protein ubiquitination during ubiquitin-dependent protein degradation, regulation of protein degradation tagging activity, regulation of protein ubiquitination during ubiquitin-dependent protein catabolic process Subtypes: regulation of proteasomal ubiquitin-dependent protein catabolic process [GO:0032434], negative regulation of ubiquitin-dependent protein catabolic process [GO:2000059], positive regulation of ubiquitin-dependent protein catabolic process [GO:2000060]